{
  "term_id": "GO:0006338",
  "gene_symbol": "YEATS2",
  "gene_name": "YEATS domain-containing protein 2",
  "term_label": "chromatin remodeling",
  "gene": "UniProtKB:Q9ULM3"
}